{
  "gene_name": "Tubulin alpha-3D chain",
  "term_label": "microtubule",
  "gene": "UniProtKB:P0DPH8",
  "gene_symbol": "TUBA3D",
  "term_id": "GO:0005874"
}